regulation of vernalization response [GO:0010219] (biological process) Relationships: is a type of regulation of response to stress [GO:0080134]; regulates vernalization response [GO:0010048] Sources: GOC:sm Subtypes: positive regulation of vernalization response [GO:0010220], negative regulation of vernalization response [GO:0010221] Definition: Any process that modulates the frequency, rate or extent of the vernalization response, by which induction of flowering is normally caused by extended exposure to cold temperatures.